dihydrobenzophenanthridine oxidase activity [GO:0047132] (molecular function) Definition: Catalysis of the reaction: O2 + dihydrosanguinarine = H2O2 + sanguinarine. Relationships: is a type of oxidoreductase activity, acting on the CH-NH group of donors, oxygen as acceptor [GO:0016647] Sources: EC:1.5.3.12 Also known as: dihydrobenzophenanthridine:oxygen oxidoreductase activity